regulation of maintenance of mitotic sister chromatid cohesion, centromeric [GO:2000718] (biological process) Also known as: regulation of maintenance of centromeric mitotic sister chromatin cohesion, regulation of maintenance of mitotic sister chromatin cohesion at centromere, regulation of maintenance of sister chromatin cohesion at centromere at mitosis Subtypes: negative regulation of maintenance of mitotic sister chromatid cohesion, centromeric [GO:2000719], positive regulation of maintenance of mitotic sister chromatid cohesion, centromeric [GO:2000720] Definition: Any process that modulates the frequency, rate or extent of maintenance of mitotic sister chromatid cohesion in the centromeric region. Relationships: is_a regulation of maintenance of mitotic sister chromatid cohesion [GO:0034182]; is a type of regulation of centromeric sister chromatid cohesion [GO:0070602]; regulates maintenance of mitotic sister chromatid cohesion, centromeric [GO:0071960] Sources: GOC:mah